{
  "term_id": "UNKNOWN:0002",
  "gene_symbol": "OSBPL7",
  "gene": "UniProtKB:Q9BZF2",
  "term_label": "Unknown biological process",
  "gene_name": "Oxysterol-binding protein-related protein 7"
}